cellular response to caffeine [GO:0071313] (biological process) Sources: GOC:mah Definition: Any process that results in a change in state or activity of a cell (in terms of movement, secretion, enzyme production, gene expression, etc.) as a result of a caffeine stimulus. Caffeine is an alkaloid found in numerous plant species, where it acts as a natural pesticide that paralyzes and kills certain insects feeding upon them. Relationships: is a type of response to caffeine [GO:0031000]; is a type of cellular response to alkaloid [GO:0071312]; is_a cellular response to purine-containing compound [GO:0071415] Regulation: negatively regulated by GO:1901181